{
  "term_id": "GO:0005886",
  "term_label": "plasma membrane",
  "gene": "UniProtKB:P51575",
  "gene_name": "P2X purinoceptor 1",
  "gene_symbol": "P2RX1"
}